intermediate mesoderm structural organization [GO:0048402] (biological process) Sources: GOC:dgh Also known as: intermediate mesoderm structural organisation Relationships: is a type of mesoderm structural organization [GO:0048338]; is part of intermediate mesoderm morphogenesis [GO:0048390] Definition: The process that contributes to the act of creating the structural organization of the intermediate mesoderm. This process pertains to the physical shaping of a rudimentary structure.